negative regulation of antigen processing and presentation of peptide antigen via MHC class I [GO:0002590] (BP) Subtypes: GO:1904283 Also known as: down regulation of antigen processing and presentation of peptide antigen via MHC class I, down-regulation of antigen processing and presentation of peptide antigen via MHC class I, downregulation of antigen processing and presentation of peptide antigen via MHC class I, negative regulation of peptide antigen processing and presentation via MHC class I, inhibition of antigen processing and presentation of peptide antigen via MHC class I Sources: GOC:add Relationships: is a type of negative regulation of antigen processing and presentation of peptide antigen [GO:0002584]; is a type of regulation of antigen processing and presentation of peptide antigen via MHC class I [GO:0002589]; negatively regulates GO:0002474 Definition: Any process that stops, prevents, or reduces the frequency, rate, or extent of antigen processing and presentation of peptide antigen via MHC class I.